transmembrane collagen trimer [GO:0030936] (cellular component) Subtypes: GO:0005600, collagen type XVII trimer [GO:0030937], collagen type XXIII trimer [GO:1990322], collagen type XXV trimer [GO:1990327] Also known as: MACIT References: PMID:21421911 Relationships: is a type of collagen trimer [GO:0005581]; is a type of plasma membrane protein complex [GO:0098797] Definition: Any collagen trimer that passes through a lipid bilayer membrane.